negative regulation of intrinsic apoptotic signaling pathway in response to DNA damage [GO:1902230] (biological process) References: PMID:15314165 Sources: GOC:BHF, GOC:TermGenie, GOC:mtg_apoptosis, GOC:rl Definition: Any process that stops, prevents or reduces the frequency, rate or extent of intrinsic apoptotic signaling pathway in response to DNA damage. Also known as: down regulation of intrinsic apoptotic signaling pathway in response to DNA damage, down-regulation of intrinsic apoptotic signaling pathway in response to DNA damage, downregulation of intrinsic apoptotic signaling pathway in response to DNA damage, inhibition of intrinsic apoptotic signaling pathway in response to DNA damage, down regulation of DNA damage response, signal transduction resulting in induction of apoptosis, down-regulation of DNA damage response, signal transduction resulting in induction of apoptosis, downregulation of DNA damage response, signal transduction resulting in induction of apoptosis, inhibition of DNA damage response, signal transduction resulting in induction of apoptosis, negative regulation of DNA damage response, signal transduction resulting in induction of apoptosis Relationships: is a type of regulation of intrinsic apoptotic signaling pathway in response to DNA damage [GO:1902229]; is a type of negative regulation of intrinsic apoptotic signaling pathway [GO:2001243]; negatively regulates GO:0008630 Subtypes: negative regulation of intrinsic apoptotic signaling pathway in response to DNA damage by p53 class mediator [GO:1902166]